{
  "gene_symbol": "VEZF1",
  "gene": "UniProtKB:Q14119",
  "term_id": "GO:0000981",
  "gene_name": "Vascular endothelial zinc finger 1",
  "term_label": "DNA-binding transcription factor activity, RNA polymerase II-specific"
}